nuclear vitamin D receptor binding [GO:0042809] (molecular function) Relationships: is a type of nuclear receptor binding [GO:0016922] Definition: Binding to a nuclear vitamin D receptor, a nuclear receptor that mediates the action of vitamin D by binding DNA and controlling the transcription of hormone-sensitive genes. References: PMID:12637589 Sources: GOC:jl Also known as: vitamin D receptor binding, VDR binding, calciferol receptor binding